{
  "term_id": "GO:0061844",
  "gene_name": "C-X-C motif chemokine 13",
  "gene": "UniProtKB:O43927",
  "term_label": "antimicrobial humoral immune response mediated by antimicrobial peptide",
  "gene_symbol": "CXCL13"
}